cupric reductase (NADH) activity [GO:0008823] (molecular function) Definition: Catalysis of the reaction: 2 Cu2+ + NADH = 2 Cu+ + H+ + NAD+. References: PMID:10510271 Sources: RHEA:66848 Relationships: is_a oxidoreductase activity, acting on metal ions, NAD or NADP as acceptor [GO:0016723]